{
  "gene_name": "Zinc finger protein 586",
  "term_id": "GO:0000978",
  "gene_symbol": "ZNF586",
  "term_label": "RNA polymerase II cis-regulatory region sequence-specific DNA binding",
  "gene": "UniProtKB:Q9NXT0"
}